dimeric IgA immunoglobulin complex [GO:0071750] (cellular component) Subtypes: secretory dimeric IgA immunoglobulin complex [GO:0071752] Also known as: dimeric IgA antibody, dimeric IgA1 antibody Definition: A protein complex composed of two monomeric IgA immunoglobulin complexes linked through both direct disulfide bonds and through a disulfide binded monomer of J chain acting as a bridge. Each IgA monomer consists of two identical immunoglobulin heavy chains of an IgA isotype and two identical immunoglobulin light chains, held together by disulfide bonds. Dimeric IgA is sometimes complexed additionally with secretory component, and present in the extracellular space, in mucosal areas or other tissues, or circulating in the blood or lymph. Note: Note that an IgA immunoglobulin complex has the function of antigen binding if a suitable antigen is available. Dimeric IgA is by far the most common form of polymeric IgA. In human only the IgA1 isotype is capable of a dimeric form. Relationships: is_a polymeric IgA immunoglobulin complex [GO:0071749] References: PMID:16362985 Sources: GOC:add, ISBN:0781765196